{
  "term_label": "Unknown biological process",
  "gene": "UniProtKB:P60866",
  "gene_name": "Small ribosomal subunit protein uS10",
  "term_id": "UNKNOWN:0002",
  "gene_symbol": "RPS20"
}